{
  "term_label": "plasma membrane",
  "gene": "UniProtKB:Q96JA1",
  "gene_name": "Leucine-rich repeats and immunoglobulin-like domains protein 1",
  "gene_symbol": "LRIG1",
  "term_id": "GO:0005886"
}